{
  "gene_symbol": "CNTROB",
  "gene_name": "Centrobin",
  "term_id": "GO:0051299",
  "term_label": "centrosome separation",
  "gene": "UniProtKB:Q8N137"
}